{
  "gene": "UniProtKB:P59665",
  "term_id": "GO:0050829",
  "gene_name": "Neutrophil defensin 1",
  "gene_symbol": "DEFA1B",
  "term_label": "defense response to Gram-negative bacterium"
}